{
  "gene": "UniProtKB:Q8N8U9",
  "term_id": "GO:0001568",
  "gene_symbol": "BMPER",
  "term_label": "blood vessel development",
  "gene_name": "BMP-binding endothelial regulator protein"
}